{
  "gene": "UniProtKB:Q96HP0",
  "term_label": "guanyl-nucleotide exchange factor activity",
  "gene_name": "Dedicator of cytokinesis protein 6",
  "gene_symbol": "DOCK6",
  "term_id": "GO:0005085"
}